{
  "gene_symbol": "TMCO4",
  "term_label": "Unknown cellular component",
  "gene_name": "Transmembrane and coiled-coil domain-containing protein 4",
  "term_id": "UNKNOWN:0003",
  "gene": "UniProtKB:Q5TGY1"
}